{
  "term_id": "UNKNOWN:0001",
  "gene_symbol": "KCTD7",
  "gene": "UniProtKB:Q96MP8",
  "term_label": "Unknown molecular function",
  "gene_name": "BTB_POZ domain-containing protein KCTD7"
}